{
  "gene_symbol": "ZSWIM9",
  "gene": "UniProtKB:Q86XI8",
  "term_label": "Unknown cellular component",
  "term_id": "UNKNOWN:0003",
  "gene_name": "Uncharacterized protein ZSWIM9"
}